negative regulation of response to reactive oxygen species [GO:1901032] (biological process) Subtypes: negative regulation of removal of superoxide radicals [GO:1904832] Definition: Any process that stops, prevents or reduces the frequency, rate or extent of response to reactive oxygen species. Sources: GOC:TermGenie, GOC:kmv Relationships: is_a regulation of response to reactive oxygen species [GO:1901031]; is a type of negative regulation of response to oxidative stress [GO:1902883]; negatively regulates GO:0000302 Also known as: down regulation of response to AOS, down regulation of response to ROI, down regulation of response to ROS, down regulation of response to active oxygen species, down regulation of response to reactive oxidative species, down regulation of response to reactive oxygen intermediate, down regulation of response to reactive oxygen species, down-regulation of response to AOS, down-regulation of response to ROI, down-regulation of response to ROS, down-regulation of response to active oxygen species, down-regulation of response to reactive oxidative species, down-regulation of response to reactive oxygen intermediate, down-regulation of response to reactive oxygen species, downregulation of response to AOS, downregulation of response to ROI, downregulation of response to ROS, downregulation of response to active oxygen species, downregulation of response to reactive oxidative species, downregulation of response to reactive oxygen intermediate, downregulation of response to reactive oxygen species, inhibition of response to AOS, inhibition of response to ROI, inhibition of response to ROS, inhibition of response to active oxygen species, inhibition of response to reactive oxidative species, inhibition of response to reactive oxygen intermediate, negative regulation of response to AOS, negative regulation of response to ROI, negative regulation of response to ROS, negative regulation of response to active oxygen species, negative regulation of response to reactive oxidative species, negative regulation of response to reactive oxygen intermediate, inhibition of response to reactive oxygen species